L-amino-acid oxidase activity [GO:0001716] (molecular function) Subtypes: L-aspartate oxidase activity [GO:0008734], L-lysine 6-oxidase activity [GO:0033736], L-glutamate oxidase activity [GO:0050025], L-lysine oxidase activity [GO:0050029], L-phenylalaine oxidase activity [GO:0106329] Sources: RHEA:13781 Also known as: L-amino-acid:oxygen oxidoreductase (deaminating), ophio-amino-acid oxidase activity Definition: Catalysis of the reaction: an L-alpha-amino acid + H2O + O2 = a 2-oxocarboxylate + H2O2 + NH4+. Relationships: is a type of primary methylamine oxidase activity [GO:0008131]